nexine [GO:0043672] (cellular component) Note: Note that nexine is distinguished on purely morphological criteria; compare with 'endexine ; GO:0043671'. See also 'sexine ; GO:0043673'. Definition: The inner, non-sculptured part of the exine which lies below the sexine. References: PMID:5722147 Relationships: is a type of GO:0110165; is part of exine [GO:0043668]